dendritic tree [GO:0097447] (cellular component) Relationships: is a type of neuron projection [GO:0043005]; is part of somatodendritic compartment [GO:0036477]; has part GO:0030425 Sources: GOC:aruk, GOC:bc, NIF_Subcellular:sao172297168 Definition: The entire complement of dendrites for a neuron, consisting of each primary dendrite and all its branches.